{
  "term_label": "Unknown molecular function",
  "term_id": "UNKNOWN:0001",
  "gene_name": "Uncharacterized protein C14orf178",
  "gene_symbol": "C14orf178",
  "gene": "UniProtKB:Q8N769"
}